{
  "gene_name": "Olfactory receptor 4S1",
  "gene_symbol": "OR4S1",
  "gene": "UniProtKB:Q8NGB4",
  "term_label": "plasma membrane",
  "term_id": "GO:0005886"
}